response to copper ion [GO:0046688] (biological process) Sources: GOC:ai Definition: Any process that results in a change in state or activity of a cell or an organism (in terms of movement, secretion, enzyme production, gene expression, etc.) as a result of a copper ion stimulus. Relationships: is a type of response to metal ion [GO:0010038] Subtypes: cellular response to copper ion [GO:0071280], stress response to copper ion [GO:1990169] Also known as: response to copper, copper sensitivity/resistance